histone H3K9 dimethyltransferase activity [GO:0140942] (molecular function) Note: Comment: Note that the residue position corresponds to the canonical human H3 histone (UniProtKB:P84243); this residue is conserved across all eukaryotes. Residue 1 is the first residue following removal of the initiating Methionine (Met). Note that each histone is encoded by multiple genes, and sequences may vary across different genes within an organism. Relationships: is_a GO:0046974 Sources: RHEA:64444 Also known as: histone H3-K9 dimethylation, histone H3K9 dimethylation, histone H3K9 dimethylase activity, histone H3K9 mono/dimethylase activity, histone lysine N-dimethyltransferase activity (H3-K9 specific) Definition: Catalysis of the reaction: L-lysyl9-[histone H3] + 2 S-adenosyl-L-methionine = 2 H+ + N6,N6-dimethyl-L-lysyl9-[histone H3] + 2 S-adenosyl-L-homocysteine. This reaction is the successive addition of two methyl groups to the unmethylated lysine residue at position 9 of histone H3, producing histone H3K9me2.